{
  "term_id": "GO:0017154",
  "gene_symbol": "PLXNB3",
  "gene_name": "Plexin-B3",
  "term_label": "semaphorin receptor activity",
  "gene": "UniProtKB:Q9ULL4"
}